coenzyme F420-0:L-glutamate ligase activity [GO:0052618] (molecular function) Definition: Catalysis of the reaction: GTP + L-glutamate + factor F420-0 = GDP + H+ + factor gamma-F420-1 + phosphate. Relationships: is a type of coenzyme F420-0 gamma-glutamyl ligase activity [GO:0043773] Sources: MetaCyc:RXN-8080